{
  "gene_name": "Complement receptor type 2",
  "gene": "UniProtKB:P20023",
  "term_label": "extracellular space",
  "gene_symbol": "CR2",
  "term_id": "GO:0005615"
}